{
  "gene": "UniProtKB:P12838",
  "gene_symbol": "DEFA4",
  "term_id": "GO:0140911",
  "gene_name": "Defensin alpha 4",
  "term_label": "pore-forming activity"
}